{
  "term_label": "Cul2-RING ubiquitin ligase complex",
  "gene_symbol": "PRAMEF7",
  "term_id": "GO:0031462",
  "gene_name": "PRAME family member 7",
  "gene": "UniProtKB:Q5VXH5"
}